{
  "gene": "UniProtKB:Q96AC6",
  "term_label": "ATP hydrolysis activity",
  "gene_symbol": "KIFC2",
  "term_id": "GO:0016887",
  "gene_name": "Kinesin-like protein KIFC2"
}